{
  "gene_name": "Krueppel-like factor 14",
  "term_id": "GO:0000981",
  "term_label": "DNA-binding transcription factor activity, RNA polymerase II-specific",
  "gene_symbol": "KLF14",
  "gene": "UniProtKB:Q8TD94"
}